{
  "gene": "UniProtKB:Q8N4B1",
  "gene_symbol": "PHETA1",
  "term_id": "GO:0005769",
  "gene_name": "Sesquipedalian-1",
  "term_label": "early endosome"
}